{
  "term_id": "GO:0045944",
  "term_label": "positive regulation of transcription by RNA polymerase II",
  "gene_name": "Myocyte-specific enhancer factor 2C",
  "gene_symbol": "MEF2C",
  "gene": "UniProtKB:Q06413"
}